low-affinity basic amino acid transmembrane transporter activity [GO:0097625] (molecular function) Relationships: is a type of GO:0015174 Also known as: low affinity basic amino acid transmembrane transporter activity Definition: Enables the transfer of basic amino acids from one side of a membrane to the other. Basic amino acids have a pH above 7. In low-affinity transport the transporter is able to bind the solute only if it is present at very high concentrations. Subtypes: low-affinity L-arginine transmembrane transporter activity [GO:0097626] Sources: GOC:pr